{
  "gene": "UniProtKB:Q9H0X4",
  "term_label": "cell surface",
  "term_id": "GO:0009986",
  "gene_name": "Protein FAM234A",
  "gene_symbol": "FAM234A"
}